{
  "term_label": "ribosomal large subunit biogenesis",
  "gene_name": "Ribosome biogenesis regulatory protein homolog",
  "term_id": "GO:0042273",
  "gene_symbol": "RRS1",
  "gene": "UniProtKB:Q15050"
}